{
  "gene_name": "U11_U12 small nuclear ribonucleoprotein 48 kDa protein",
  "gene": "UniProtKB:Q6IEG0",
  "gene_symbol": "SNRNP48",
  "term_label": "U12-type spliceosomal complex",
  "term_id": "GO:0005689"
}